{
  "term_id": "GO:0048019",
  "gene_name": "Dickkopf-related protein 1",
  "gene": "UniProtKB:O94907",
  "term_label": "receptor antagonist activity",
  "gene_symbol": "DKK1"
}